{
  "gene_name": "Gilles de la Tourette syndrome chromosomal region candidate gene 1 protein",
  "term_id": "UNKNOWN:0001",
  "gene_symbol": "GTSCR1",
  "gene": "UniProtKB:Q86UQ5",
  "term_label": "Unknown molecular function"
}